{
  "term_label": "positive regulation of epidermal growth factor receptor signaling pathway",
  "term_id": "GO:0045742",
  "gene_symbol": "SHKBP1",
  "gene": "UniProtKB:Q8TBC3",
  "gene_name": "SH3KBP1-binding protein 1"
}